{
  "gene_name": "Paraspeckle component 1",
  "gene_symbol": "PSPC1",
  "term_label": "RNA binding",
  "term_id": "GO:0003723",
  "gene": "UniProtKB:Q8WXF1"
}